NADH-dependent peroxiredoxin activity [GO:0102039] (MF) Also known as: alkylhydroperoxide reductase activity References: PMID:12517450 Sources: GOC:pz, RHEA:62628 Definition: Catalysis of the reaction: a hydroperoxide + H+ + NADH = an alcohol + H2O + NAD+. Relationships: is a type of peroxiredoxin activity [GO:0051920]